formation of structure involved in a symbiotic process [GO:0044111] (biological process) Subtypes: development of symbiont in host [GO:0044114], formation of specialized structure for nutrient acquisition [GO:0052093], initiation of appressorium formation [GO:0075025], appressorium maturation [GO:0075035], GO:0075039 Also known as: development on or near surface of other organism involved in symbiotic interaction, development during symbiotic interaction, development involved in symbiotic interaction, development of symbiont during interaction with host, development of symbiont involved in interaction with host, development on or near surface of other organism during symbiotic interaction Sources: GO:jl, GOC:pamgo_curators Relationships: is_a biological process involved in interspecies interaction between organisms [GO:0044419] Regulation: regulated by GO:0044145; negatively regulated by negative regulation of formation of structure involved in a symbiotic process [GO:0044147]; positively regulated by GO:0044149 Definition: The progression of an organism from an initial condition to a later condition, occurring when the organism is in a symbiotic interaction.